aldehyde biosynthetic process [GO:0046184] (biological process) Relationships: is a type of aldehyde metabolic process [GO:0006081]; is a type of biosynthetic process [GO:0009058] Subtypes: GO:0006634, methylglyoxal biosynthetic process [GO:0019242], aldosterone biosynthetic process [GO:0032342], GO:0042189, pyridoxal biosynthetic process [GO:0042821], pyridoxal phosphate biosynthetic process [GO:0042823], glyceraldehyde-3-phosphate biosynthetic process [GO:0046166], acetaldehyde biosynthetic process [GO:0046186], GO:0046293, GO:0140876, chanoclavine-I aldehyde biosynthetic process [GO:1900569], GO:1900994, glyoxal biosynthetic process [GO:1903191] Also known as: aldehyde anabolism, aldehyde biosynthesis, aldehyde formation, aldehyde synthesis Definition: The chemical reactions and pathways resulting in the formation of aldehydes, any organic compound with the formula R-CH=O. Sources: GOC:ai